{
  "gene_symbol": "PARD3",
  "term_label": "cell adhesion",
  "term_id": "GO:0007155",
  "gene_name": "Partitioning defective 3 homolog",
  "gene": "UniProtKB:Q8TEW0"
}